{
  "term_label": "cytoplasm",
  "gene_symbol": "RNF167",
  "term_id": "GO:0005737",
  "gene": "UniProtKB:Q9H6Y7",
  "gene_name": "E3 ubiquitin-protein ligase RNF167"
}